{
  "gene_symbol": "TLR3",
  "gene_name": "Toll-like receptor 3",
  "term_label": "plasma membrane",
  "gene": "UniProtKB:O15455",
  "term_id": "GO:0005886"
}